{
  "gene": "UniProtKB:Q96ST8",
  "gene_symbol": "CEP89",
  "term_label": "mitochondrion organization",
  "term_id": "GO:0007005",
  "gene_name": "Centrosomal protein of 89 kDa"
}